{
  "term_id": "UNKNOWN:0002",
  "gene": "UniProtKB:A0A075B6Y3",
  "term_label": "Unknown biological process",
  "gene_name": "T cell receptor alpha joining 3",
  "gene_symbol": "TRAJ3"
}